{
  "term_label": "proteasome-mediated ubiquitin-dependent protein catabolic process",
  "gene": "UniProtKB:Q9BVQ7",
  "gene_name": "ATPase family gene 2 protein homolog B",
  "term_id": "GO:0043161",
  "gene_symbol": "AFG2B"
}